{
  "gene": "UniProtKB:Q6DRA6",
  "gene_symbol": "H2BC19P",
  "term_id": "GO:0061844",
  "gene_name": "Putative histone H2B type 2-D",
  "term_label": "antimicrobial humoral immune response mediated by antimicrobial peptide"
}